positive regulation of ubiquinone biosynthetic process [GO:1904775] (biological process) Definition: Any process that activates or increases the frequency, rate or extent of ubiquinone biosynthetic process. Also known as: positive regulation of coenzyme Q biosynthesis, positive regulation of coenzyme Q biosynthetic process, positive regulation of ubiquinone anabolism, positive regulation of ubiquinone biosynthesis, positive regulation of ubiquinone formation, positive regulation of ubiquinone synthesis, up regulation of coenzyme Q biosynthesis, up regulation of coenzyme Q biosynthetic process, up regulation of ubiquinone anabolism, up regulation of ubiquinone biosynthesis, up regulation of ubiquinone biosynthetic process, up regulation of ubiquinone formation, up regulation of ubiquinone synthesis, up-regulation of coenzyme Q biosynthesis, up-regulation of coenzyme Q biosynthetic process, up-regulation of ubiquinone anabolism, up-regulation of ubiquinone biosynthesis, up-regulation of ubiquinone biosynthetic process, up-regulation of ubiquinone formation, up-regulation of ubiquinone synthesis, upregulation of coenzyme Q biosynthesis, upregulation of coenzyme Q biosynthetic process, upregulation of ubiquinone anabolism, upregulation of ubiquinone biosynthesis, upregulation of ubiquinone biosynthetic process, upregulation of ubiquinone formation, upregulation of ubiquinone synthesis, activation of coenzyme Q biosynthesis, activation of coenzyme Q biosynthetic process, activation of coenzyme Q10 biosynthesis, activation of coenzyme Q10 biosynthetic process, activation of coenzyme Q6 biosynthesis, activation of coenzyme Q6 biosynthetic process, activation of coenzyme Q8 biosynthesis, activation of coenzyme Q8 biosynthetic process, activation of coenzyme Q9 biosynthesis, activation of coenzyme Q9 biosynthetic process, activation of ubiquinone anabolism, activation of ubiquinone biosynthesis, activation of ubiquinone biosynthetic process, activation of ubiquinone formation, activation of ubiquinone synthesis, positive regulation of coenzyme Q10 biosynthesis, positive regulation of coenzyme Q10 biosynthetic process, positive regulation of coenzyme Q6 biosynthesis, positive regulation of coenzyme Q6 biosynthetic process, positive regulation of coenzyme Q8 biosynthesis, positive regulation of coenzyme Q8 biosynthetic process, positive regulation of coenzyme Q9 biosynthesis, positive regulation of coenzyme Q9 biosynthetic process, up regulation of coenzyme Q10 biosynthesis, up regulation of coenzyme Q10 biosynthetic process, up regulation of coenzyme Q6 biosynthesis, up regulation of coenzyme Q6 biosynthetic process, up regulation of coenzyme Q8 biosynthesis, up regulation of coenzyme Q8 biosynthetic process, up regulation of coenzyme Q9 biosynthesis, up regulation of coenzyme Q9 biosynthetic process, up-regulation of coenzyme Q10 biosynthesis, up-regulation of coenzyme Q10 biosynthetic process, up-regulation of coenzyme Q6 biosynthesis, up-regulation of coenzyme Q6 biosynthetic process, up-regulation of coenzyme Q8 biosynthesis, up-regulation of coenzyme Q8 biosynthetic process, up-regulation of coenzyme Q9 biosynthesis, up-regulation of coenzyme Q9 biosynthetic process, upregulation of coenzyme Q10 biosynthesis, upregulation of coenzyme Q10 biosynthetic process, upregulation of coenzyme Q6 biosynthesis, upregulation of coenzyme Q6 biosynthetic process, upregulation of coenzyme Q8 biosynthesis, upregulation of coenzyme Q8 biosynthetic process, upregulation of coenzyme Q9 biosynthesis, upregulation of coenzyme Q9 biosynthetic process Relationships: is a type of GO:0009891; is a type of GO:0010795; is a type of positive regulation of small molecule metabolic process [GO:0062013]; positively regulates GO:0006744 References: PMID:8125303 Sources: GOC:TermGenie, GO_REF:0000058